regulation of regulatory ncRNA-mediated heterochromatin formation [GO:0010964] (BP) Sources: GOC:dph, GOC:tb Also known as: regulation of RNAi-mediated heterochromatin assembly, regulation of ncRNA-mediated heterochromatin formation, regulation of chromatin silencing by small RNA, regulation of heterochromatin assembly by small RNA, regulation of small non-coding RNA-mediated heterochromatin formation Relationships: is a type of regulation of heterochromatin formation [GO:0031445]; is a type of regulation of gene silencing by regulatory ncRNA [GO:0060966]; regulates regulatory ncRNA-mediated heterochromatin formation [GO:0031048] Subtypes: negative regulation of regulatory ncRNA-mediated heterochromatin formation [GO:0060906], regulation of siRNA-mediated facultative heterochromatin formation [GO:1902802] Definition: Any process that modulates the frequency, rate or extent of small non-coding RNA-mediated heterochromatin formation.